{
  "gene": "UniProtKB:O14974",
  "gene_name": "Protein phosphatase 1 regulatory subunit 12A",
  "gene_symbol": "PPP1R12A",
  "term_label": "neuron projection morphogenesis",
  "term_id": "GO:0048812"
}